mitotic spindle [GO:0072686] (cellular component) Definition: A spindle that forms as part of mitosis. Mitotic and meiotic spindles contain distinctive complements of proteins associated with microtubules. References: PMID:11408572, PMID:18367542, PMID:8027178 Sources: GOC:mah, GOC:vw Relationships: is a type of GO:0005819